{
  "gene": "UniProtKB:Q9UK12",
  "gene_symbol": "ZNF222",
  "term_label": "Unknown biological process",
  "term_id": "UNKNOWN:0002",
  "gene_name": "Zinc finger protein 222"
}